{
  "gene_symbol": "PRR11",
  "term_label": "Unknown molecular function",
  "gene": "UniProtKB:Q96HE9",
  "gene_name": "Proline-rich protein 11",
  "term_id": "UNKNOWN:0001"
}